geranylgeranylglycerol-phosphate geranylgeranyltransferase activity [GO:0047295] (molecular function) Definition: Catalysis of the reaction: (2E,6E,10E)-geranylgeranyl diphosphate + sn-3-O-(geranylgeranyl)glycerol 1-phosphate = 2,3-bis-O-(geranylgeranyl)-sn-glycerol 1-phosphate + diphosphate. References: PMID:15356000, PMID:16494480 Sources: RHEA:18109 Also known as: (S)-2,3-di-O-geranylgeranylglyceryl phosphate synthase activity, DGGGP synthase activity, geranylgeranyl diphosphate:sn-3-O-(geranylgeranyl)glycerol 1-phosphate geranylgeranyltransferase activity, geranylgeranyloxyglycerol phosphate geranylgeranyltransferase activity, geranylgeranyltransferase II Note: This function is involved in archaeal lipid synthesis. Relationships: is a type of prenyltransferase activity [GO:0004659]